proprioception [GO:0019230] (biological process) Sources: ISBN:072168677X Definition: The series of events by which an organism senses the position, location, orientation, and movement of the body and its parts. Proprioception is mediated by proprioceptors, sensory nerve terminals found in muscles, tendons, and joint capsules, which give information concerning movements and position of the body. The receptors in the labyrinth are sometimes also considered proprioceptors. Relationships: is a type of sensory perception [GO:0007600]; is part of GO:0050884 Subtypes: perception of static position [GO:0019231], perception of rate of movement [GO:0019232], proprioception involved in equilibrioception [GO:0051355]